{
  "gene": "UniProtKB:Q5TYW2",
  "term_label": "Unknown molecular function",
  "term_id": "UNKNOWN:0001",
  "gene_name": "Ankyrin repeat domain-containing protein 20A1",
  "gene_symbol": "ANKRD20A1"
}